{
  "term_label": "Unknown biological process",
  "gene_symbol": "MCCC1",
  "term_id": "UNKNOWN:0002",
  "gene_name": "Methylcrotonoyl-CoA carboxylase subunit alpha, mitochondrial",
  "gene": "UniProtKB:Q96RQ3"
}